{
  "gene": "UniProtKB:B4DS77",
  "gene_symbol": "SHISA9",
  "gene_name": "Protein shisa-9",
  "term_id": "GO:0045211",
  "term_label": "postsynaptic membrane"
}